{
  "term_id": "GO:0030334",
  "gene": "UniProtKB:O15520",
  "gene_name": "Fibroblast growth factor 10",
  "gene_symbol": "FGF10",
  "term_label": "regulation of cell migration"
}